{
  "gene_name": "Olfactory receptor 2T10",
  "gene": "UniProtKB:Q8NGZ9",
  "term_id": "GO:0050911",
  "gene_symbol": "OR2T10",
  "term_label": "detection of chemical stimulus involved in sensory perception of smell"
}